{
  "term_label": "Unknown molecular function",
  "gene": "UniProtKB:Q3KNS1",
  "term_id": "UNKNOWN:0001",
  "gene_name": "Patched domain-containing protein 3",
  "gene_symbol": "PTCHD3"
}